positive regulation of bone mineralization involved in bone maturation [GO:1900159] (BP) Also known as: up regulation of bone mineralization involved in bone maturation, up-regulation of bone mineralization involved in bone maturation, upregulation of bone mineralization involved in bone maturation, activation of bone mineralization involved in bone maturation Sources: GOC:BHF, GOC:TermGenie Relationships: is a type of positive regulation of bone mineralization [GO:0030501]; is a type of regulation of bone mineralization involved in bone maturation [GO:1900157]; positively regulates GO:0035630 Definition: Any process that activates or increases the frequency, rate or extent of bone mineralization involved in bone maturation.